{
  "gene_name": "Caprin-2",
  "term_label": "positive regulation of canonical Wnt signaling pathway",
  "gene_symbol": "CAPRIN2",
  "gene": "UniProtKB:Q6IMN6",
  "term_id": "GO:0090263"
}